{
  "gene_symbol": "KCNK3",
  "term_id": "GO:0005886",
  "term_label": "plasma membrane",
  "gene_name": "Potassium channel subfamily K member 3",
  "gene": "UniProtKB:O14649"
}